{
  "term_label": "cytoplasm",
  "gene": "UniProtKB:Q9H0R4",
  "term_id": "GO:0005737",
  "gene_symbol": "HDHD2",
  "gene_name": "Haloacid dehalogenase-like hydrolase domain-containing protein 2"
}